regulation of early endosome to late endosome transport [GO:2000641] (biological process) Sources: GOC:BHF Definition: Any process that modulates the frequency, rate or extent of early endosome to late endosome transport. Subtypes: GO:2000642, positive regulation of early endosome to late endosome transport [GO:2000643] Relationships: is a type of regulation of intracellular transport [GO:0032386]; is a type of regulation of vesicle-mediated transport [GO:0060627]; regulates early endosome to late endosome transport [GO:0045022]